{
  "term_id": "GO:0055090",
  "gene_name": "Apolipoprotein E",
  "gene_symbol": "APOE",
  "term_label": "acylglycerol homeostasis",
  "gene": "UniProtKB:P02649"
}